{
  "term_id": "GO:0043005",
  "gene_symbol": "CYFIP2",
  "term_label": "neuron projection",
  "gene_name": "Cytoplasmic FMR1-interacting protein 2",
  "gene": "UniProtKB:Q96F07"
}